biological process involved in interaction with symbiont [GO:0051702] (biological process) Also known as: interaction with symbiont Subtypes: detection of symbiont [GO:0009602], acquisition of nutrients from symbiont [GO:0051850], translocation of molecules into symbiont [GO:0051862], GO:0051873, formation by host of specialized structure for nutrient acquisition from symbiont [GO:0052098], lectin-induced modified bacterial internalization [GO:0106136] Definition: An interaction between two organisms living together in more or less intimate association. The term symbiont is used for the smaller (macro) of the two members of a symbiosis; the various forms of symbiosis include parasitism, commensalism and mutualism. Relationships: is a type of biological process involved in symbiotic interaction [GO:0044403] Sources: GOC:cc